{
  "gene_name": "Aspartoacylase",
  "gene_symbol": "ASPA",
  "term_id": "UNKNOWN:0002",
  "gene": "UniProtKB:P45381",
  "term_label": "Unknown biological process"
}